chloride-activated potassium channel activity [GO:0070089] (molecular function) Definition: Enables the transmembrane transfer of a potassium cation by a channel that opens when a chloride ion has been bound by the channel complex or one of its constituent parts. Sources: GOC:kmv, GOC:mtg_transport Relationships: is a type of potassium channel activity [GO:0005267]; is_a GO:0022839; is_a ligand-gated monoatomic cation channel activity [GO:0099094]